detection of disaccharide stimulus [GO:0034288] (biological process) Relationships: is a type of detection of carbohydrate stimulus [GO:0009730]; is_a GO:0034285 Sources: GOC:sart Definition: The series of events in which a stimulus from a disaccharide is received and converted into a molecular signal. Subtypes: detection of sucrose stimulus [GO:0009731], detection of maltose stimulus [GO:0034289] Also known as: perception of disaccharide stimulus